{
  "term_id": "GO:0035312",
  "gene_name": "5' exonuclease Apollo",
  "term_label": "5'-3' DNA exonuclease activity",
  "gene_symbol": "DCLRE1B",
  "gene": "UniProtKB:Q9H816"
}